negative regulation of renal output by angiotensin [GO:0003083] (biological process) Definition: The process in which angiotensin directly decreases the rate of natriuresis and diuresis in the kidney. Also known as: angiotensin mediated negative regulation of renal output, angiotensin-mediated negative regulation of renal output Relationships: is a type of regulation of renal output by angiotensin [GO:0002019]; is a type of positive regulation of systemic arterial blood pressure [GO:0003084] Sources: GOC:dph, GOC:mtg_cardio, GOC:tb Subtypes: negative regulation of glomerular filtration by angiotensin [GO:0003106], GO:0035820